{
  "gene": "UniProtKB:Q6PCB6",
  "term_id": "GO:1902817",
  "term_label": "negative regulation of protein localization to microtubule",
  "gene_symbol": "ABHD17C",
  "gene_name": "Alpha_beta hydrolase domain-containing protein 17C"
}